endoplasmic reticulum membrane biogenesis [GO:0160031] (biological process) Definition: The process in which an endoplasmic reticulum membrane is synthesized, aggregates, and bonds together. References: PMID:19825355, PMID:24373967, PMID:34617598 Relationships: is a type of membrane biogenesis [GO:0044091]; is part of GO:0090158 Also known as: ER membrane biogenesis